{
  "gene": "UniProtKB:Q86YS3",
  "gene_name": "Rab11 family-interacting protein 4",
  "term_id": "GO:0032456",
  "term_label": "endocytic recycling",
  "gene_symbol": "RAB11FIP4"
}